{
  "term_label": "ciliary basal body",
  "term_id": "GO:0036064",
  "gene_name": "Tubulin polyglutamylase TTLL13",
  "gene": "UniProtKB:A6NNM8",
  "gene_symbol": "TTLL13"
}